genkwanin 4'-O-methyltransferase activity [GO:0102533] (molecular function) Definition: Catalysis of the reaction: genkwanin + S-adenosyl-L-methionine = apigenin 4',7-dimethyl ether + S-adenosyl-L-homocysteine. Relationships: is a type of GO:0008168 Sources: RHEA:73263